{
  "term_id": "GO:0038187",
  "gene": "UniProtKB:Q9NR96",
  "gene_symbol": "TLR9",
  "term_label": "pattern recognition receptor activity",
  "gene_name": "Toll-like receptor 9"
}